{
  "gene_symbol": "ZNF664",
  "gene": "UniProtKB:Q8N3J9",
  "term_label": "Unknown cellular component",
  "gene_name": "Zinc finger protein 664",
  "term_id": "UNKNOWN:0003"
}